{
  "term_label": "N-formyl peptide receptor activity",
  "gene_name": "Probable G-protein coupled receptor 32",
  "gene": "UniProtKB:O75388",
  "gene_symbol": "GPR32",
  "term_id": "GO:0004982"
}